bronchiole development [GO:0060435] (biological process) Sources: GOC:dph, GOC:mtg_lung Definition: The biological process whose specific outcome is the progression of a bronchiole from an initial condition to its mature state. This process begins with the formation of the bronchiole and ends with the mature structure. A bronchiole is the first airway branch that no longer contains cartilage; it is a branch of the bronchi. Relationships: is a type of GO:0030323; is part of GO:0030324